response to paracetamol [GO:1901554] (biological process) Relationships: is a type of GO:1901698; is a type of response to oxygen-containing compound [GO:1901700] Also known as: response to acetaminophen Sources: GOC:TermGenie Definition: Any process that results in a change in state or activity of a cell or an organism (in terms of movement, secretion, enzyme production, gene expression, etc.) as a result of a paracetamol stimulus.